{
  "term_label": "Unknown molecular function",
  "term_id": "UNKNOWN:0001",
  "gene_name": "Cytochrome c oxidase subunit 6B1",
  "gene_symbol": "COX6B1",
  "gene": "UniProtKB:P14854"
}